{
  "term_label": "Unknown cellular component",
  "gene": "UniProtKB:Q92562",
  "gene_symbol": "FIG4",
  "gene_name": "Polyphosphoinositide phosphatase",
  "term_id": "UNKNOWN:0003"
}